{
  "gene_symbol": "OLIG3",
  "gene": "UniProtKB:Q7RTU3",
  "term_label": "positive regulation of transcription by RNA polymerase II",
  "term_id": "GO:0045944",
  "gene_name": "Oligodendrocyte transcription factor 3"
}